{
  "gene": "UniProtKB:K7EIQ3",
  "term_id": "UNKNOWN:0001",
  "gene_symbol": "ZNF561-AS1",
  "gene_name": "Uncharacterized protein ZNF561-AS1",
  "term_label": "Unknown molecular function"
}